{
  "gene_symbol": "IGHD2OR15-2B",
  "term_label": "Unknown biological process",
  "gene": "UniProtKB:A0A075B7B9",
  "term_id": "UNKNOWN:0002",
  "gene_name": "Protein IGHD2OR15-2A (Fragment)"
}